regulation of pentose-phosphate shunt [GO:0043456] (biological process) Definition: Any process that modulates the frequency, rate or extent of the pentose-phosphate shunt, the process in which glucose is oxidized, coupled to NADPH synthesis. Subtypes: negative regulation of pentose-phosphate shunt [GO:1905856], positive regulation of pentose-phosphate shunt [GO:1905857] Also known as: regulation of pentose phosphate pathway, regulation of pentose phosphate shunt, regulation of pentose-phosphate pathway Relationships: is a type of regulation of amide metabolic process [GO:0034248]; is a type of regulation of generation of precursor metabolites and energy [GO:0043467]; is a type of regulation of carbohydrate catabolic process [GO:0043470]; is a type of regulation of NADP metabolic process [GO:1902031]; regulates pentose-phosphate shunt [GO:0006098] Sources: GOC:jl